mannosamine catabolic process [GO:0046346] (biological process) Subtypes: N-acetylmannosamine catabolic process [GO:0006053] Relationships: is a type of amino sugar catabolic process [GO:0046348] Also known as: mannosamine breakdown, mannosamine catabolism, mannosamine degradation Definition: The chemical reactions and pathways resulting in the breakdown of mannosomine, 2-amino-2-deoxymannose; the D-isomer is a constituent of neuraminic acids as well as mucolipids and mucoproteins. Sources: GOC:curators